{
  "gene_symbol": "LINC00474",
  "term_label": "Unknown biological process",
  "term_id": "UNKNOWN:0002",
  "gene": "UniProtKB:Q9P2X8",
  "gene_name": "Putative uncharacterized protein encoded by LINC00474"
}